(R)-2-hydroxyglutarate (NAD+) dehydrogenase activity [GO:0120568] (molecular function) Also known as: 2-oxoglutarate reductase activity Relationships: is a type of oxidoreductase activity, acting on the CH-OH group of donors, NAD or NADP as acceptor [GO:0016616]; is a type of (R)-2-hydroxyglutarate dehydrogenase activity [GO:0051990] Definition: Catalysis of the reaction: (R)-2-hydroxyglutarate + NAD+ = 2-oxoglutarate + NADH + H+. References: PMID:26774271 Sources: RHEA:49612